endoplasmic reticulum to Golgi vesicle-mediated transport [GO:0006888] (biological process) Definition: The directed movement of substances from the endoplasmic reticulum (ER) to the Golgi, mediated by COP II vesicles. Small COP II coated vesicles form from the ER and then fuse directly with the cis-Golgi. Larger structures are transported along microtubules to the cis-Golgi. Also known as: ER to Golgi transport, ER to Golgi vesicle-mediated transport, anterograde (ER to Golgi) transport, anterograde transport, ER to Golgi, anterograde transport, endoplasmic reticulum to Golgi, anterograde vesicle-mediated transport, ER to Golgi, anterograde vesicle-mediated transport, endoplasmic reticulum to Golgi, endoplasmic reticulum to Golgi transport, rough ER to cis-Golgi transport, rough ER to cis-Golgi vesicle-mediated transport, rough endoplasmic reticulum to cis-Golgi transport, rough endoplasmic reticulum to cis-Golgi vesicle-mediated transport Relationships: is_a intracellular transport [GO:0046907]; is_a GO:0048193; occurs in cytoplasm [GO:0005737] Sources: GOC:ascb_2009, GOC:dph, GOC:jp, GOC:tb, ISBN:0716731363 Regulation: regulated by GO:0060628; RO_0002213 by positive regulation of ER to Golgi vesicle-mediated transport [GO:1902953]